{
  "term_id": "GO:0005178",
  "term_label": "integrin binding",
  "gene_name": "Integrin beta-8",
  "gene_symbol": "ITGB8",
  "gene": "UniProtKB:P26012"
}